{
  "gene": "UniProtKB:Q8WZ74",
  "term_id": "GO:0098978",
  "gene_symbol": "CTTNBP2",
  "term_label": "glutamatergic synapse",
  "gene_name": "Cortactin-binding protein 2"
}